very-low-density lipoprotein particle receptor binding [GO:0070326] (molecular function) Also known as: VLDL receptor binding, VLDLR binding, very-low-density lipoprotein receptor binding, apolipoprotein E receptor binding Sources: GOC:BHF, GOC:mah Relationships: is a type of lipoprotein particle receptor binding [GO:0070325] Definition: Binding to a very-low-density lipoprotein receptor.